{
  "gene_name": "Dehydrogenase_reductase SDR family member 13",
  "term_id": "GO:0016491",
  "gene_symbol": "DHRS13",
  "gene": "UniProtKB:Q6UX07",
  "term_label": "oxidoreductase activity"
}